{
  "term_id": "GO:0034685",
  "gene": "UniProtKB:P18564",
  "gene_symbol": "ITGB6",
  "gene_name": "Integrin beta-6",
  "term_label": "integrin alphav-beta6 complex"
}